{
  "gene_name": "Protein FAM246B",
  "term_label": "Unknown biological process",
  "term_id": "UNKNOWN:0002",
  "gene_symbol": "FAM246B",
  "gene": "UniProtKB:A0A494C0N9"
}